{
  "gene_symbol": "ZNF891",
  "term_label": "RNA polymerase II transcription regulatory region sequence-specific DNA binding",
  "gene": "UniProtKB:A8MT65",
  "gene_name": "Zinc finger protein 891",
  "term_id": "GO:0000977"
}